{
  "term_id": "GO:0032040",
  "gene_name": "Ribosome biogenesis protein BMS1 homolog",
  "gene": "UniProtKB:Q14692",
  "gene_symbol": "BMS1",
  "term_label": "small-subunit processome"
}